{
  "gene_name": "Amelogenin, X isoform",
  "term_id": "GO:0070166",
  "gene": "UniProtKB:Q99217",
  "gene_symbol": "AMELX",
  "term_label": "enamel mineralization"
}